{
  "gene_symbol": "CNPY2",
  "gene_name": "Protein canopy homolog 2",
  "term_id": "UNKNOWN:0001",
  "term_label": "Unknown molecular function",
  "gene": "UniProtKB:Q9Y2B0"
}